protein K11-linked deubiquitination [GO:0035871] (biological process) Also known as: protein K11-linked deubiquitinylation, protein K11-linked deubiquitylation Relationships: is a type of protein deubiquitination [GO:0016579] Definition: A protein deubiquitination process in which a K11-linked ubiquitin chain, i.e. a polymer of ubiquitin formed by linkages between lysine residues at position 11 of the ubiquitin monomers, is removed from a protein. References: PMID:21596315 Sources: GOC:sp